{
  "gene": "UniProtKB:A6NK44",
  "gene_symbol": "GLOD5",
  "gene_name": "Glyoxalase domain-containing protein 5",
  "term_id": "UNKNOWN:0002",
  "term_label": "Unknown biological process"
}